COPII-coated ER to Golgi transport vesicle [GO:0030134] (cellular component) References: PMID:11252894, PMID:17499046, PMID:22160157, PMID:8004676 Sources: Wikipedia:COPII Also known as: COPII-associated ER to Golgi transport vesicle, COPII-associated vesicle, COPII-coated vesicle, COPII vesicle, ER to Golgi constitutive secretory pathway transport vesicle, ER to Golgi transport vesicle, ER-Golgi transport vesicle, endoplasmic reticulum to Golgi transport vesicle, endoplasmic reticulum-Golgi transport vesicle Relationships: is a type of coated vesicle [GO:0030135] Definition: A vesicle with a coat formed of the COPII coat complex proteins. The COPII coat complex is formed by the Sec23p/Sec24p and the Sec13p/Sec31p heterodimers. COPII-associated vesicles transport proteins from the rough endoplasmic reticulum to the Golgi apparatus (anterograde transport).